{
  "term_id": "UNKNOWN:0001",
  "term_label": "Unknown molecular function",
  "gene_name": "Putative uncharacterized protein SPART-AS1",
  "gene": "UniProtKB:P0CW21",
  "gene_symbol": "SPART-AS1"
}